indolylacetyl-myo-inositol galactosyltransferase activity [GO:0047227] (molecular function) Definition: Catalysis of the reaction: 1L-1-O-(indol-3-yl)acetyl-myo-inositol + UDP-D-galactose = 5-O-(indol-3-ylacetyl)-myo-inositol D-galactoside + H+ + UDP. Also known as: UDP-galactose:(indol-3-yl)acetyl-myo-inositol 5-O-D-galactosyltransferase activity, UDP-galactose:indol-3-ylacetyl-myo-inositol 5-O-D-galactosyltransferase activity, indol-3-ylacetyl-myo-inositol galactoside synthase activity, uridine diphosphogalactose-indolylacetylinositol galactosyltransferase activity Relationships: is a type of UDP-galactosyltransferase activity [GO:0035250] Sources: EC:2.4.1.156, RHEA:21148